{
  "gene_symbol": "NUDT16",
  "gene": "UniProtKB:Q96DE0",
  "term_label": "snoRNA binding",
  "gene_name": "U8 snoRNA-decapping enzyme",
  "term_id": "GO:0030515"
}